leaf development [GO:0048366] (biological process) Relationships: is a type of GO:0048827 Sources: GOC:go_curators Regulation: negatively regulated by negative regulation of leaf development [GO:1905622]; positively regulated by positive regulation of leaf development [GO:1905623]; regulated by GO:2000024 Definition: The process whose specific outcome is the progression of the leaf over time, from its formation to the mature structure. Subtypes: cotyledon development [GO:0048825]